{
  "gene_symbol": "BAX",
  "term_label": "mitochondrial fusion",
  "gene": "UniProtKB:Q07812",
  "gene_name": "Apoptosis regulator BAX",
  "term_id": "GO:0008053"
}